{
  "term_id": "GO:1904262",
  "gene_name": "KICSTOR subunit 2",
  "term_label": "negative regulation of TORC1 signaling",
  "gene_symbol": "KICS2",
  "gene": "UniProtKB:Q96MD2"
}